{
  "gene": "UniProtKB:O43615",
  "gene_name": "Mitochondrial import inner membrane translocase subunit TIM44",
  "gene_symbol": "TIMM44",
  "term_id": "GO:0005743",
  "term_label": "mitochondrial inner membrane"
}